{
  "gene_name": "COMM domain-containing protein 5",
  "gene": "UniProtKB:Q9GZQ3",
  "term_label": "nucleus",
  "term_id": "GO:0005634",
  "gene_symbol": "COMMD5"
}